plant-type cell wall [GO:0009505] (cellular component) Sources: ISBN:0471245208 Relationships: is_a cell wall [GO:0005618] Definition: A more or less rigid structure lying outside the cell membrane of a cell and composed of cellulose and pectin and other organic and inorganic substances. Subtypes: primary cell wall [GO:0009530], secondary cell wall [GO:0009531] Also known as: cellulose and pectin-containing cell wall, plant cell wall